{
  "gene_name": "Cytoplasmic dynein 1 intermediate chain 2",
  "term_id": "GO:0005868",
  "gene": "UniProtKB:Q13409",
  "gene_symbol": "DYNC1I2",
  "term_label": "cytoplasmic dynein complex"
}